{
  "term_label": "cell morphogenesis",
  "gene_symbol": "NCKAP1L",
  "gene": "UniProtKB:P55160",
  "term_id": "GO:0000902",
  "gene_name": "Nck-associated protein 1-like"
}